negative regulation of endocrocin biosynthetic process [GO:1900668] (biological process) Relationships: is a type of GO:0062014; is a type of negative regulation of secondary metabolite biosynthetic process [GO:1900377]; is a type of GO:1900667; negatively regulates endocrocin biosynthetic process [GO:1900602] Also known as: down regulation of endocrocin anabolism, down regulation of endocrocin biosynthesis, down regulation of endocrocin biosynthetic process, down regulation of endocrocin formation, down regulation of endocrocin synthesis, down-regulation of endocrocin anabolism, down-regulation of endocrocin biosynthesis, down-regulation of endocrocin biosynthetic process, down-regulation of endocrocin formation, down-regulation of endocrocin synthesis, downregulation of endocrocin anabolism, downregulation of endocrocin biosynthesis, downregulation of endocrocin biosynthetic process, downregulation of endocrocin formation, downregulation of endocrocin synthesis, inhibition of endocrocin anabolism, inhibition of endocrocin biosynthesis, inhibition of endocrocin formation, inhibition of endocrocin synthesis, negative regulation of endocrocin anabolism, negative regulation of endocrocin biosynthesis, negative regulation of endocrocin formation, negative regulation of endocrocin synthesis, inhibition of endocrocin biosynthetic process Definition: Any process that stops, prevents or reduces the frequency, rate or extent of endocrocin biosynthetic process. Sources: GOC:TermGenie, GOC:di